{
  "gene_symbol": "CALML4",
  "gene": "UniProtKB:Q96GE6",
  "term_label": "cytoplasm",
  "gene_name": "Calmodulin-like protein 4",
  "term_id": "GO:0005737"
}